{
  "gene": "UniProtKB:O00442",
  "term_id": "UNKNOWN:0002",
  "gene_name": "RNA 3'-terminal phosphate cyclase",
  "gene_symbol": "RTCA",
  "term_label": "Unknown biological process"
}